metencephalon development [GO:0022037] (biological process) Definition: The process whose specific outcome is the progression of the metencephalon over time, from its formation to the mature structure. Sources: GOC:cls, GOC:curators, GOC:dgh, GOC:dph, GOC:jid Relationships: is_a GO:0048856; BFO_0000050 hindbrain development [GO:0030902]